{
  "gene_name": "Histone H2B type W-T",
  "term_label": "nucleosome",
  "gene_symbol": "H2BW1",
  "gene": "UniProtKB:Q7Z2G1",
  "term_id": "GO:0000786"
}